{
  "gene": "UniProtKB:O75528",
  "term_label": "transcription coactivator activity",
  "gene_name": "Transcriptional adapter 3",
  "term_id": "GO:0003713",
  "gene_symbol": "TADA3"
}